{
  "gene": "UniProtKB:Q9NYY8",
  "gene_name": "FAST kinase domain-containing protein 2, mitochondrial",
  "term_label": "ribonucleoprotein granule",
  "gene_symbol": "FASTKD2",
  "term_id": "GO:0035770"
}